{
  "term_label": "Unknown biological process",
  "gene_name": "Leucine-rich repeat-containing protein 38",
  "gene": "UniProtKB:Q5VT99",
  "gene_symbol": "LRRC38",
  "term_id": "UNKNOWN:0002"
}